{
  "gene_name": "PRAME family member 5",
  "gene": "UniProtKB:Q5TYX0",
  "gene_symbol": "PRAMEF5",
  "term_id": "GO:0005737",
  "term_label": "cytoplasm"
}